{
  "gene_symbol": "PI4KAP1",
  "gene_name": "Putative inactive phosphatidylinositol 4-kinase alpha-like protein P1",
  "term_id": "UNKNOWN:0001",
  "gene": "UniProtKB:Q8N8J0",
  "term_label": "Unknown molecular function"
}